coenzyme F420-0 gamma-glutamyl ligase activity [GO:0043773] (molecular function) Subtypes: coenzyme F420-0:L-glutamate ligase activity [GO:0052618], coenzyme F420-1:gamma-L-glutamate ligase activity [GO:0052619] Also known as: F420-0 gamma-glutamyl ligase activity Definition: Catalysis of the reactions: (1) GTP + F420-0 + L-glutamate = GDP + phosphate + F420-1, and (2) GTP + F420-1 + L-glutamate = GDP + phosphate + gamma-F420-2. This is the GTP-dependent successive addition of two L-glutamates to the L-lactyl phosphodiester of 7,8-didemethyl-8-hydroxy-5-deazariboflavin (F420-0) to form F420-0-glutamyl-glutamate (F420-2), with a gamma-linkage between the two glutamates. Relationships: is a type of acid-amino acid ligase activity [GO:0016881]; has part coenzyme F420-0:L-glutamate ligase activity [GO:0052618]; has part coenzyme F420-1:gamma-L-glutamate ligase activity [GO:0052619] References: PMID:17669425